negative regulation of gastric emptying [GO:0120061] (biological process) Relationships: is a type of negative regulation of digestive system process [GO:0060457]; is_a regulation of gastric emptying [GO:0120060]; negatively regulates gastric emptying [GO:0035483] Definition: Any process that decreases the frequency, rate or extent of any gastric emptying process, the process in which the liquid and liquid-suspended solid contents of the stomach exit through the pylorus into the duodenum. References: PMID:15890336 Sources: GOC:sl